{
  "term_label": "pseudouridine synthase activity",
  "term_id": "GO:0009982",
  "gene_name": "Mitochondrial mRNA pseudouridine synthase RPUSD3",
  "gene": "UniProtKB:Q6P087",
  "gene_symbol": "RPUSD3"
}